inner cell mass cellular morphogenesis [GO:0001828] (biological process) Definition: The morphogenesis of cells in the inner cell mass. Sources: GOC:dph, ISBN:0124020607, ISBN:0198542771 Note: See also the Anatomical Dictionary for Mouse Development ontology terms 'TS4, inner cell mass ; EMAP:14' and 'TS5, inner cell mass ; EMAP:24'. Relationships: is a type of cell morphogenesis [GO:0000902]; is a type of embryonic morphogenesis [GO:0048598]; BFO_0000050 GO:0001826